positive regulation of unidimensional cell growth [GO:0051512] (biological process) Also known as: up regulation of unidimensional cell growth, up-regulation of unidimensional cell growth, upregulation of unidimensional cell growth, activation of unidimensional cell growth, positive regulation of cell elongation, stimulation of unidimensional cell growth Relationships: is_a positive regulation of cell morphogenesis [GO:0010770]; is a type of positive regulation of cell growth [GO:0030307]; is_a positive regulation of developmental growth [GO:0048639]; is a type of regulation of unidimensional cell growth [GO:0051510]; positively regulates unidimensional cell growth [GO:0009826] Sources: GOC:ai Subtypes: GO:0051515, positive regulation of bipolar cell growth [GO:0051518] Definition: Any process that activates or increases the frequency, rate or extent of unidimensional cell growth, the process in which a cell irreversibly increases in size in one [spatial] dimension or along one axis.